protein phosphatase binding [GO:0019903] (molecular function) Sources: GOC:jl Subtypes: GO:0008157, GO:0030346, GO:0051721, GO:1990634 Definition: Binding to a protein phosphatase. Relationships: is_a phosphatase binding [GO:0019902]